negative regulation of vascular permeability [GO:0043116] (biological process) Also known as: down regulation of vascular permeability, down-regulation of vascular permeability, downregulation of vascular permeability, inhibition of vascular permeability Subtypes: negative regulation of blood-brain barrier permeability [GO:1905604] Definition: Any process that reduces the extent to which blood vessels can be pervaded by fluid. Relationships: is a type of GO:0043114 Sources: GOC:jl